{
  "term_id": "GO:0015721",
  "gene": "UniProtKB:Q9Y6L6",
  "gene_name": "Solute carrier organic anion transporter family member 1B1",
  "term_label": "bile acid and bile salt transport",
  "gene_symbol": "SLCO1B1"
}